vascular associated smooth muscle cell apoptotic process [GO:1905288] (biological process) Also known as: VSMC apoptotic process, vascular smooth muscle cell apoptotic process, VSMC apoptosis, vascular associated smooth muscle cell apoptosis, vascular smooth muscle cell apoptosis Definition: Any apoptotic process in a vascular associated smooth muscle cell. References: PMID:26493107 Sources: GOC:BHF, GOC:BHF_miRNA, GOC:TermGenie, GOC:rph, GO_REF:0000085 Relationships: is a type of GO:0034390 Regulation: RO_0002211 by regulation of vascular associated smooth muscle cell apoptotic process [GO:1905459]; negatively regulated by negative regulation of vascular associated smooth muscle cell apoptotic process [GO:1905460]; RO_0002213 by GO:1905461